{
  "term_id": "UNKNOWN:0002",
  "gene_name": "Testis-expressed sequence 37 protein",
  "gene": "UniProtKB:Q96LM6",
  "gene_symbol": "TEX37",
  "term_label": "Unknown biological process"
}